{
  "gene_name": "Taste receptor type 2 member 9",
  "term_label": "membrane",
  "gene": "UniProtKB:Q9NYW1",
  "gene_symbol": "TAS2R9",
  "term_id": "GO:0016020"
}